host cell synaptic vesicle membrane [GO:0098585] (cellular component) Sources: GOC:dos Relationships: is a type of host cell cytoplasmic vesicle membrane [GO:0044162]; is part of host cell synaptic vesicle [GO:0098584] Definition: The lipid bilayer surrounding a host synaptic vesicle.